{
  "term_id": "GO:0005634",
  "gene": "UniProtKB:Q3SY56",
  "gene_name": "Transcription factor Sp6",
  "term_label": "nucleus",
  "gene_symbol": "SP6"
}